{
  "gene_symbol": "FASTK",
  "gene": "UniProtKB:Q14296",
  "term_id": "GO:0005759",
  "term_label": "mitochondrial matrix",
  "gene_name": "Fas-activated serine_threonine kinase"
}